{
  "gene_symbol": "LIN7B",
  "gene": "UniProtKB:Q9HAP6",
  "gene_name": "Protein lin-7 homolog B",
  "term_label": "MPP7-DLG1-LIN7 complex",
  "term_id": "GO:0097025"
}